RNA polymerase II general transcription initiation factor activity [GO:0016251] (molecular function) References: PMID:10384286, PMID:10747032, PMID:23442138, PMID:25693126 Sources: GOC:txnOH-2018 Definition: A general transcription initiation factor activity that contributes to transcription start site selection and transcription initiation of genes transcribed by RNA polymerase II. The general transcription factors for RNA polymerase II include TFIIB, TFIID, TFIIE, TFIIF, TFIIH and TATA-binding protein (TBP). In most species, RNA polymerase II transcribes all messenger RNAs (mRNAs), most untranslated regulatory RNAs, the majority of the snoRNAs, four of the five snRNAs (U1, U2, U4, and U5), and other small noncoding RNAs. For some small RNAs there is variability between species as to whether it is transcribed by RNA polymerase II or RNA polymerase III. However there are also rare exceptions, such as Trypanosoma brucei, where RNA polymerase I transcribes certain mRNAs in addition to its normal role in rRNA transcription. Also known as: GTF2 activity, basal RNA polymerase II transcription factor activity, general RNA polymerase II transcription factor activity, RNA polymerase II core promoter sequence-specific DNA binding transcription factor activity, RNA polymerase II core promoter sequence-specific DNA binding transcription factor activity involved in preinitiation complex assembly, sequence-specific core promoter binding RNA polymerase II transcription factor activity involved in preinitiation complex assembly, transcription factor activity, RNA polymerase II core promoter sequence-specific DNA binding, transcription factor activity, RNA polymerase II core promoter sequence-specific binding involved in preinitiation complex assembly Relationships: is a type of general transcription initiation factor activity [GO:0140223]; is part of transcription by RNA polymerase II [GO:0006366] Note: General transcription factors assemble with the RNA polymerase at promoter DNA to form the pre-initiation complex (PIC), bind to and open promoter DNA, initiate RNA synthesis and stimulate the escape of the polymerase from the promoter. Not all subunits of the general transcription factor are necessarily present in all promoters to initiate transcription. The distinction between general transcription factors and DNA-binding transcription factors is that the latter modulate the selection of which genes are expressed under specific conditions, while general transcription factors belong to the constitutive machinery required for transcription to occur.